{
  "gene_name": "Methyltransferase-like protein 25B",
  "term_id": "UNKNOWN:0001",
  "gene_symbol": "METTL25B",
  "term_label": "Unknown molecular function",
  "gene": "UniProtKB:Q96FB5"
}